{
  "term_label": "mitochondrion",
  "term_id": "GO:0005739",
  "gene_symbol": "GLRX2",
  "gene_name": "Glutaredoxin-2, mitochondrial",
  "gene": "UniProtKB:Q9NS18"
}